estradiol 6-beta-monooxygenase activity [GO:0047882] (molecular function) Definition: Catalysis of the reaction: AH(2) + estradiol-17beta + O2 = 6beta-hydroxyestradiol-17beta + A + H2O. Sources: EC:1.14.99.11, RHEA:19137 Also known as: estradiol 6b-hydroxylase activity, estradiol 6b-monooxygenase activity, estradiol 6-beta-hydroxylase activity, estradiol 6beta-hydroxylase activity, estradiol 6beta-monooxygenase activity, estradiol-17beta,hydrogen-donor:oxygen oxidoreductase (6beta-hydroxylating) Relationships: is a type of steroid hydroxylase activity [GO:0008395]; is a type of GO:0016705